{
  "term_label": "cyclin-dependent protein serine/threonine kinase activator activity",
  "gene_symbol": "CKS1B",
  "term_id": "GO:0061575",
  "gene_name": "Cyclin-dependent kinases regulatory subunit 1",
  "gene": "UniProtKB:P61024"
}